{
  "gene_name": "Potassium voltage-gated channel subfamily E member 4",
  "gene": "UniProtKB:Q8WWG9",
  "term_label": "potassium ion export across plasma membrane",
  "gene_symbol": "KCNE4",
  "term_id": "GO:0097623"
}